{
  "term_id": "GO:0005160",
  "term_label": "transforming growth factor beta receptor binding",
  "gene_name": "Muellerian-inhibiting factor",
  "gene": "UniProtKB:P03971",
  "gene_symbol": "AMH"
}